neuroligin clustering involved in postsynaptic membrane assembly [GO:0097118] (biological process) Relationships: is a type of receptor clustering [GO:0043113]; BFO_0000050 postsynaptic membrane assembly [GO:0097104] Also known as: Nlgn clustering, neuroligin clustering, postsynaptic neuroligin clustering Definition: The receptor clustering process involved in assembly of the postsynaptic membrane in which neuroligins are localized to distinct domains in the cell membrane. Neuroligins are neuronal cell surface proteins on the postsynaptic membrane that mediate synapse formation between neurons. References: PMID:12796785 Sources: GOC:BHF, GOC:sjp